{
  "gene_symbol": "CCDC169",
  "term_label": "Unknown molecular function",
  "gene": "UniProtKB:A6NNP5",
  "gene_name": "Coiled-coil domain-containing protein 169",
  "term_id": "UNKNOWN:0001"
}